{
  "term_label": "Unknown biological process",
  "term_id": "UNKNOWN:0002",
  "gene_symbol": "SPDYE3",
  "gene": "UniProtKB:A6NKU9",
  "gene_name": "Speedy protein E3"
}